anaerobic lactate catabolic process [GO:1990485] (biological process) Definition: The chemical reactions and pathways resulting in the breakdown of lactate (2-hydroxypropanoic acid) in the absence of oxygen. References: PMID:11133436 Sources: GOC:mengo_curators Also known as: anaerobic lactic acid catabolic process Relationships: is a type of GO:1903457